{
  "term_label": "protein-folding chaperone binding",
  "gene": "UniProtKB:Q9UNE7",
  "gene_symbol": "STUB1",
  "term_id": "GO:0051087",
  "gene_name": "E3 ubiquitin-protein ligase CHIP"
}